{
  "gene": "UniProtKB:P08581",
  "gene_symbol": "MET",
  "term_label": "neuron differentiation",
  "term_id": "GO:0030182",
  "gene_name": "Hepatocyte growth factor receptor"
}